{
  "term_label": "single-stranded RNA binding",
  "gene_symbol": "DHX58",
  "term_id": "GO:0003727",
  "gene_name": "ATP-dependent RNA helicase DHX58",
  "gene": "UniProtKB:Q96C10"
}